{
  "term_id": "GO:0032452",
  "gene": "UniProtKB:Q6ZMT4",
  "term_label": "histone demethylase activity",
  "gene_name": "Lysine-specific demethylase 7A",
  "gene_symbol": "KDM7A"
}